L-asparagine import across plasma membrane [GO:1903811] (biological process) References: PMID:23895341 Sources: GOC:TermGenie, GO_REF:0000075 Also known as: asparagine import, L-asparagine import into cell Definition: The directed movement of L-asparagine from outside of a cell, across the plasma membrane and into the cytosol. Relationships: is a type of asparagine transport [GO:0006867]; is a type of organic cation transport [GO:0015695]; is a type of amino acid import across plasma membrane [GO:0089718]; is a type of L-alpha-amino acid transmembrane transport [GO:1902475]; is a type of asparagine transmembrane transport [GO:1903713]